{
  "term_id": "GO:0045087",
  "gene_name": "E3 ubiquitin-protein ligase TRIM15",
  "gene": "UniProtKB:Q9C019",
  "gene_symbol": "TRIM15",
  "term_label": "innate immune response"
}